antigen processing and presentation of exogenous peptide antigen via MHC class I [GO:0042590] (biological process) Definition: The process in which an antigen-presenting cell expresses a peptide antigen of exogenous origin on its cell surface in association with an MHC class I protein complex. The peptide antigen is typically, but not always, processed from a whole protein. Class I here refers to classical class I molecules. References: PMID:15771591 Sources: GOC:add, ISBN:0781735149 Also known as: cross presentation, cross priming, cross-presentation, cross-priming, antigen presentation, exogenous antigen via MHC class I, antigen presentation, exogenous antigen via major histocompatibility complex class I, exogenous peptide antigen processing and presentation via MHC class I Relationships: is a type of antigen processing and presentation of peptide antigen via MHC class I [GO:0002474]; is_a GO:0002478 Subtypes: antigen processing and presentation of exogenous peptide antigen via MHC class I, TAP-dependent [GO:0002479], antigen processing and presentation of exogenous peptide antigen via MHC class I, TAP-independent [GO:0002480]